{
  "term_id": "GO:0000981",
  "gene_symbol": "BHLHA9",
  "term_label": "DNA-binding transcription factor activity, RNA polymerase II-specific",
  "gene": "UniProtKB:Q7RTU4",
  "gene_name": "Class A basic helix-loop-helix protein 9"
}